{
  "term_id": "GO:0006606",
  "gene_name": "Nuclear pore complex protein Nup88",
  "term_label": "protein import into nucleus",
  "gene": "UniProtKB:Q99567",
  "gene_symbol": "NUP88"
}